chronic inflammatory response to non-antigenic stimulus [GO:0002545] (biological process) Regulation: RO_0002211 by regulation of chronic inflammatory response to non-antigenic stimulus [GO:0002880]; negatively regulated by negative regulation of chronic inflammatory response to non-antigenic stimulus [GO:0002881]; positively regulated by positive regulation of chronic inflammatory response to non-antigenic stimulus [GO:0002882] Definition: A chronic inflammatory response to a non-antigenic stimulus such as heat or physical trauma. Sources: GOC:jal Relationships: is a type of chronic inflammatory response [GO:0002544]